{
  "term_id": "UNKNOWN:0003",
  "gene": "UniProtKB:A0A1B0GVH7",
  "term_label": "Unknown cellular component",
  "gene_symbol": "IQCM",
  "gene_name": "IQ domain-containing protein M"
}